{
  "gene_symbol": "LGALS3",
  "term_label": "extracellular space",
  "gene_name": "Galectin-3",
  "gene": "UniProtKB:P17931",
  "term_id": "GO:0005615"
}